{
  "gene_name": "11-beta-hydroxysteroid dehydrogenase type 2",
  "term_id": "GO:0008211",
  "gene": "UniProtKB:P80365",
  "term_label": "glucocorticoid metabolic process",
  "gene_symbol": "HSD11B2"
}